{
  "gene_name": "Methyltransferase N6AMT1",
  "gene": "UniProtKB:Q9Y5N5",
  "gene_symbol": "HEMK2",
  "term_label": "S-adenosylmethionine-dependent methyltransferase activity",
  "term_id": "GO:0008757"
}